negative regulation of cell morphogenesis [GO:0010771] (biological process) Definition: Any process that decreases the frequency, rate or extent of cell morphogenesis contributing to cell differentiation. Cell morphogenesis involved in differentiation is the change in form (cell shape and size) that occurs when relatively unspecialized cells acquire specialized structural and/or functional features that characterize the cells, tissues, or organs of the mature organism or some other relatively stable phase of the organism's life history. Subtypes: GO:0051511, negative regulation of formation of radial glial scaffolds [GO:0061925] Sources: GOC:dph, GOC:tb Relationships: is a type of negative regulation of cell development [GO:0010721]; is a type of regulation of cell morphogenesis [GO:0022604]; negatively regulates cell morphogenesis [GO:0000902]